{
  "gene_name": "BMP-binding endothelial regulator protein",
  "term_id": "GO:0005201",
  "term_label": "extracellular matrix structural constituent",
  "gene_symbol": "BMPER",
  "gene": "UniProtKB:Q8N8U9"
}